farnesol catabolic process [GO:0016488] (biological process) Relationships: is a type of GO:0016095; is a type of GO:0016107; is a type of farnesol metabolic process [GO:0016487]; is a type of primary alcohol catabolic process [GO:0034310] Sources: GOC:go_curators Also known as: farnesol breakdown, farnesol catabolism, farnesol degradation Definition: The chemical reactions and pathways resulting in the breakdown of the sesquiterpenoid alcohol farnesol, 3,7,11-trimethyl-2,6,10,dodecatrien-1-ol.